{
  "term_label": "peptidyl-prolyl cis-trans isomerase activity",
  "gene": "UniProtKB:P68106",
  "term_id": "GO:0003755",
  "gene_name": "Peptidyl-prolyl cis-trans isomerase FKBP1B",
  "gene_symbol": "FKBP1B"
}